{
  "term_label": "Unknown molecular function",
  "gene_name": "Beta-defensin 104",
  "term_id": "UNKNOWN:0001",
  "gene": "UniProtKB:Q8WTQ1",
  "gene_symbol": "DEFB104A"
}